{
  "gene_name": "Putative neuroblastoma breakpoint family member 8",
  "gene": "UniProtKB:Q3BBV2",
  "gene_symbol": "NBPF8",
  "term_label": "Unknown molecular function",
  "term_id": "UNKNOWN:0001"
}